{
  "term_label": "phosphatidylinositol-4,5-bisphosphate binding",
  "gene_name": "FERM and PDZ domain-containing protein 4",
  "term_id": "GO:0005546",
  "gene": "UniProtKB:Q14CM0",
  "gene_symbol": "FRMPD4"
}